{
  "gene_name": "Cancer_testis antigen family 45 member A6",
  "gene": "UniProtKB:P0DMU7",
  "gene_symbol": "CT45A6",
  "term_id": "UNKNOWN:0003",
  "term_label": "Unknown cellular component"
}